{
  "term_id": "GO:0030688",
  "gene": "UniProtKB:Q96GA3",
  "gene_symbol": "LTV1",
  "gene_name": "Protein LTV1 homolog",
  "term_label": "preribosome, small subunit precursor"
}